{
  "term_id": "GO:0006508",
  "gene_name": "Disintegrin and metalloproteinase domain-containing protein 20",
  "term_label": "proteolysis",
  "gene": "UniProtKB:O43506",
  "gene_symbol": "ADAM20"
}